sterol desaturase activity [GO:0070704] (molecular function) Definition: Catalysis of the introduction of a double bond into a sterol molecule. Sources: GOC:mah, GOC:vw Relationships: is a type of oxidoreductase activity, acting on paired donors, with oxidation of a pair of donors resulting in the reduction of molecular oxygen to two molecules of water [GO:0016717] Subtypes: GO:0000248, C-22 sterol desaturase (NADPH) activity [GO:0000249], GO:0050046, cholesterol 7-desaturase [NAD(P)H] activity [GO:0170056]